cell cycle phase [GO:0022403] (biological process) Subtypes: GO:0000279, GO:0044838, G1 phase [GO:0051318], G2 phase [GO:0051319], GO:0051320, anaphase [GO:0051322], prophase [GO:0051324], interphase [GO:0051325], telophase [GO:0051326], meiotic cell cycle phase [GO:0098762], mitotic cell cycle phase [GO:0098763] Sources: GOC:mtg_cell_cycle Definition: One of the distinct periods or stages into which the cell cycle is divided. Each phase is characterized by the occurrence of specific biochemical and morphological events. Note: Note that this term should not be used for direct annotation. If you are trying to make an annotation to x phase, it is likely that the correct annotation is 'regulation of x/y phase transition' or to a process which occurs during the reported phase (i.e mitotic DNA replication for mitotic S-phase). To capture the phase when a specific location or process is observed, the phase term can be used in an annotation extension (PMID:24885854) applied to a cellular component term (with the relation exists_during) or a biological process term (with the relation happens_during). Relationships: is a type of biological phase [GO:0044848]